{
  "gene_symbol": "SYNDIG1",
  "term_id": "GO:0030672",
  "gene_name": "Synapse differentiation-inducing gene protein 1",
  "term_label": "synaptic vesicle membrane",
  "gene": "UniProtKB:Q9H7V2"
}